{
  "gene_symbol": "LMX1B",
  "gene_name": "LIM homeobox transcription factor 1-beta",
  "term_id": "GO:0000977",
  "gene": "UniProtKB:O60663",
  "term_label": "RNA polymerase II transcription regulatory region sequence-specific DNA binding"
}